{
  "term_id": "UNKNOWN:0001",
  "term_label": "Unknown molecular function",
  "gene_symbol": "PLIN5",
  "gene_name": "Perilipin-5",
  "gene": "UniProtKB:Q00G26"
}